negative regulation of D-glucose import [GO:0046325] (biological process) Sources: GOC:ai Relationships: is a type of GO:0010829; is_a GO:0046324; negatively regulates D-glucose import [GO:0046323] Also known as: down regulation of glucose import, down-regulation of glucose import, downregulation of glucose import, negative regulation of glucose import, negative regulation of glucose uptake, inhibition of glucose import Definition: Any process that stops, prevents, or reduces the frequency, rate or extent of the import of the hexose monosaccharide glucose into a cell or organelle.